oxysterol binding [GO:0008142] (MF) Relationships: is a type of sterol binding [GO:0032934] Sources: GOC:curators Definition: Binding to oxysterol, an oxidized form of cholesterol.